{
  "gene": "UniProtKB:Q96CN7",
  "gene_symbol": "ISOC1",
  "gene_name": "Isochorismatase domain-containing protein 1",
  "term_id": "GO:0005737",
  "term_label": "cytoplasm"
}